{
  "term_id": "GO:0000978",
  "gene_symbol": "CRX",
  "gene_name": "Cone-rod homeobox protein",
  "term_label": "RNA polymerase II cis-regulatory region sequence-specific DNA binding",
  "gene": "UniProtKB:O43186"
}